{
  "gene": "UniProtKB:Q53HV7",
  "term_label": "oxidized pyrimidine nucleobase lesion DNA N-glycosylase activity",
  "gene_symbol": "SMUG1",
  "gene_name": "Single-strand selective monofunctional uracil DNA glycosylase",
  "term_id": "GO:0000703"
}